{
  "term_label": "actin filament binding",
  "term_id": "GO:0051015",
  "gene_symbol": "CORO1A",
  "gene": "UniProtKB:P31146",
  "gene_name": "Coronin-1A"
}